{
  "gene_name": "bMERB domain-containing protein 1",
  "term_id": "GO:0015630",
  "gene": "UniProtKB:Q96MC5",
  "gene_symbol": "BMERB1",
  "term_label": "microtubule cytoskeleton"
}